regulation of ERK1 and ERK2 cascade [GO:0070372] (biological process) Also known as: regulation of ERK cascade, regulation of ERK1 and ERK2 signaling pathway, regulation of ERK1 and ERK2 signalling pathway, regulation of ERK1/2 cascade, regulation of ERK1 cascade, regulation of ERK2 cascade, regulation of MAPK1 cascade, regulation of MAPK3 cascade Sources: GOC:add, ISBN:0121245462, ISBN:0896039986 Definition: Any process that modulates the frequency, rate or extent of signal transduction mediated by the ERK1 and ERK2 cascade. Subtypes: negative regulation of ERK1 and ERK2 cascade [GO:0070373], positive regulation of ERK1 and ERK2 cascade [GO:0070374] Relationships: is a type of GO:0043408; regulates GO:0070371